O-phospho-L-serine:2-oxoglutarate aminotransferase activity [GO:0004648] (molecular function) Relationships: is a type of transaminase activity [GO:0008483] Definition: Catalysis of the reaction: O-phospho-L-serine + 2-oxoglutarate = 3-phosphonooxypyruvate + L-glutamate. Also known as: phosphoserine aminotransferase activity, phosphoserine transaminase activity, 3-O-phospho-L-serine:2-oxoglutarate aminotransferase activity, 3-phosphoserine aminotransferase activity, 3PHP transaminase activity, L-phosphoserine aminotransferase activity, PSAT activity, PdxC, SerC, hydroxypyruvic phosphate--glutamic transaminase activity, phosphohydroxypyruvate transaminase activity, phosphohydroxypyruvic--glutamic transaminase activity Sources: EC:2.6.1.52